{
  "term_label": "Unknown cellular component",
  "term_id": "UNKNOWN:0003",
  "gene": "UniProtKB:Q13070",
  "gene_symbol": "GAGE6",
  "gene_name": "G antigen 6"
}